carboxylic acid transport [GO:0046942] (biological process) Sources: GOC:ai Relationships: is_a organic anion transport [GO:0015711]; is a type of organic acid transport [GO:0015849] Subtypes: GO:0000101, GO:0001762, dicarboxylic acid transport [GO:0006835], tricarboxylic acid transport [GO:0006842], asparagine transport [GO:0006867], glutamine transport [GO:0006868], GO:0015718, sialic acid transport [GO:0015739], aromatic amino acid transport [GO:0015801], GO:0015803, GO:0015807, gamma-aminobutyric acid transport [GO:0015812], glycine transport [GO:0015816], ornithine transport [GO:0015822], phenylalanine transport [GO:0015823], threonine transport [GO:0015826], diaminopimelate transport [GO:0015830], alanine transport [GO:0032328], serine transport [GO:0032329], hydroxyproline transport [GO:0034589], chrysobactin transport [GO:0042932], achromobactin transport [GO:0042935], GO:0042940, homoserine transport [GO:0042968], icosanoid transport [GO:0071715], hydroxycinnamic acid transport [GO:1904952], carboxylic acid transmembrane transport [GO:1905039], ganglioside GM1 transport to membrane [GO:1905572] Definition: The directed movement of carboxylic acids into, out of or within a cell, or between cells, by means of some agent such as a transporter or pore. Carboxylic acids are organic acids containing one or more carboxyl (COOH) groups or anions (COO-).